positive regulation of serine-type endopeptidase activity [GO:1900005] (biological process) Relationships: is a type of positive regulation of endopeptidase activity [GO:0010950]; is a type of GO:1900003; positively regulates GO:0004252 Definition: Any process that activates or increases the frequency, rate or extent of serine-type endopeptidase activity. Also known as: positive regulation of blood coagulation factor activity, up regulation of blood coagulation factor activity, up regulation of serine-type endopeptidase activity Sources: GOC:TermGenie